regulation of cellular component biogenesis [GO:0044087] (biological process) Sources: GOC:jl Relationships: is a type of regulation of cellular process [GO:0050794]; regulates GO:0044085 Subtypes: regulation of actin filament bundle assembly [GO:0032231], regulation of fungal-type cell wall biogenesis [GO:0032995], regulation of protein-containing complex assembly [GO:0043254], positive regulation of cellular component biogenesis [GO:0044089], regulation of cell projection assembly [GO:0060491], regulation of linear element assembly [GO:0090006], regulation of ribosome biogenesis [GO:0090069], regulation of inclusion body assembly [GO:0090083], regulation of sphingolipid biosynthetic process [GO:0090153], regulation of synaptonemal complex assembly [GO:0090173], negative regulation of actin cortical patch assembly [GO:0120133], regulation of hyaluranon cable assembly [GO:1900104], regulation of extracellular matrix assembly [GO:1901201], GO:1901888, regulation of cell septum assembly [GO:1901891], regulation of organelle assembly [GO:1902115], regulation of ascospore-type prospore membrane formation [GO:1903023], regulation of iron-sulfur cluster assembly [GO:1903329], regulation of secondary cell septum biogenesis [GO:1903395], regulation of t-circle formation [GO:1904429], regulation of cytokinesis, actomyosin contractile ring assembly [GO:2000431], regulation of secondary cell wall biogenesis [GO:2000652], regulation of dense core granule biogenesis [GO:2000705] Definition: Any process that modulates the frequency, rate or extent of cellular component biogenesis, a process that results in the biosynthesis of constituent macromolecules, assembly, and arrangement of constituent parts of a cellular component.